{
  "term_id": "GO:0005634",
  "gene": "UniProtKB:Q9UKW6",
  "gene_name": "ETS-related transcription factor Elf-5",
  "term_label": "nucleus",
  "gene_symbol": "ELF5"
}